{
  "gene_symbol": "ZNF613",
  "gene_name": "Zinc finger protein 613",
  "gene": "UniProtKB:Q6PF04",
  "term_label": "Unknown cellular component",
  "term_id": "UNKNOWN:0003"
}